negative regulation of sodium-dependent phosphate transport [GO:2000119] (biological process) Sources: GOC:BHF Relationships: is_a negative regulation of transport [GO:0051051]; is_a GO:2000118; negatively regulates sodium-dependent phosphate transport [GO:0044341] Definition: Any process that stops, prevents, or reduces the frequency, rate or extent of sodium-dependent phosphate transport.